{
  "gene": "UniProtKB:A0A075B6Y3",
  "gene_name": "T cell receptor alpha joining 3",
  "term_id": "UNKNOWN:0001",
  "term_label": "Unknown molecular function",
  "gene_symbol": "TRAJ3"
}